pronuclear fusion [GO:0007344] (biological process) Sources: GOC:ems, ISBN:087969307X Relationships: is a type of GO:0000741; is part of GO:0007338 Definition: The merging of two pronuclei in a fertilized egg to fuse and produce a single zygotic genome.